{
  "term_id": "GO:0005634",
  "gene_name": "Ski-like protein",
  "gene_symbol": "SKIL",
  "term_label": "nucleus",
  "gene": "UniProtKB:P12757"
}